{
  "gene_name": "Sodium_potassium-transporting ATPase subunit beta-1",
  "gene": "UniProtKB:P05026",
  "gene_symbol": "ATP1B1",
  "term_id": "GO:0005890",
  "term_label": "sodium:potassium-exchanging ATPase complex"
}